negative regulation of protein K48-linked ubiquitination [GO:0061944] (biological process) Relationships: is a type of regulation of protein K48-linked ubiquitination [GO:0061945]; is a type of negative regulation of protein polyubiquitination [GO:1902915]; negatively regulates GO:0070936 Definition: Any process that stops, prevents or reduces the frequency, rate or extent of K48-linked ubiquitination, a protein ubiquitination process in which a polymer of ubiquitin, formed by linkages between lysine residues at position 48 of the ubiquitin monomers, is added to a protein. K48-linked ubiquitination targets the substrate protein for degradation. References: PMID:23460740 Sources: GOC:BHF, GOC:rph